regulation of apoptotic process in bone marrow cell [GO:0071865] (biological process) Definition: Any process that modulates the occurrence or rate of cell death by apoptotic process in the bone marrow. References: PMID:17063141 Sources: GOC:mah, GOC:mtg_apoptosis, GOC:yaf Relationships: is a type of GO:0042981; regulates apoptotic process in bone marrow cell [GO:0071839] Also known as: regulation of apoptotic process in bone marrow, regulation of apoptosis in bone marrow Subtypes: negative regulation of apoptotic process in bone marrow cell [GO:0071866], positive regulation of apoptotic process in bone marrow cell [GO:0120132]